ectoine synthase activity [GO:0033990] (molecular function) Definition: Catalysis of the reaction: N(4)-acetyl-L-2,4-diaminobutyrate = ectoine + H2O. Relationships: is a type of hydro-lyase activity [GO:0016836] Also known as: 4-N-acetyl-L-2,4-diaminobutanoate hydro-lyase (L-ectoine-forming) activity, EctC, L-ectoine synthase activity, N-acetyldiaminobutanoate dehydratase activity, N-acetyldiaminobutyrate dehydratase activity, N4-acetyl-L-2,4-diaminobutanoate hydro-lyase (L-ectoine-forming) activity Sources: EC:4.2.1.108, RHEA:17281